regulation of morphogenesis of an epithelium [GO:1905330] (biological process) References: PMID:25745997 Sources: GOC:TermGenie, GOC:bhm, GO_REF:0000058 Also known as: regulation of epithelium morphogenesis Definition: Any process that modulates the frequency, rate or extent of morphogenesis of an epithelium. Subtypes: regulation of prostatic bud formation [GO:0060685], regulation of branching involved in prostate gland morphogenesis [GO:0060687], regulation of branching involved in salivary gland morphogenesis [GO:0060693], regulation of branching involved in mammary gland duct morphogenesis [GO:0060762], regulation of branching involved in lung morphogenesis [GO:0061046], GO:0072043, regulation of branching involved in ureteric bud morphogenesis [GO:0090189], regulation of heart looping [GO:1901207], regulation of convergent extension involved in axis elongation [GO:1901232], regulation of endothelial tube morphogenesis [GO:1901509], regulation of epiboly involved in gastrulation with mouth forming second [GO:1904086], regulation of convergent extension involved in gastrulation [GO:1904103], regulation of otic vesicle morphogenesis [GO:1904118], regulation of epithelial tube formation [GO:1905276], negative regulation of morphogenesis of an epithelium [GO:1905331], GO:1905332, regulation of blood vessel branching [GO:1905553] Note: An example of this is MMRN2 in human (Q9H8L6) in PMID:25745997 (inferred from direct assay). Relationships: is a type of regulation of anatomical structure morphogenesis [GO:0022603]; regulates GO:0002009